xanthophyll biosynthetic process [GO:0016123] (biological process) Subtypes: lutein biosynthetic process [GO:0062171], spheroidene biosynthetic process [GO:1901180], capsanthin biosynthetic process [GO:1901809], astaxanthin biosynthetic process [GO:1901815], zeaxanthin biosynthetic process [GO:1901827], neoxanthin biosynthetic process [GO:1901833], GO:1901866 Definition: The chemical reactions and pathways resulting in the formation of xanthophylls, oxygen-containing carotenoids. Relationships: is a type of carotenoid biosynthetic process [GO:0016117]; is_a xanthophyll metabolic process [GO:0016122] Sources: GOC:go_curators Also known as: xanthophyll anabolism, xanthophyll biosynthesis, xanthophyll formation, xanthophyll synthesis